regulation of endothelial cell development [GO:1901550] (BP) References: PMID:19470579 Sources: GOC:TermGenie, GOC:pr Definition: Any process that modulates the frequency, rate or extent of endothelial cell development. Subtypes: negative regulation of endothelial cell development [GO:1901551], GO:1901552, regulation of establishment of endothelial barrier [GO:1903140] Relationships: is a type of regulation of endothelial cell differentiation [GO:0045601]; is a type of GO:0060284; RO_0002211 endothelial cell development [GO:0001885]